nuclear mRNA surveillance of mRNA 3'-end processing [GO:0071031] (biological process) Relationships: is a type of nuclear mRNA surveillance [GO:0071028]; has part GO:0071042 Also known as: nuclear mRNA catabolic process of mRNA with aberrant 3'-ends, nuclear mRNA quality control of mRNAs with aberrant 3'-ends Definition: The set of processes involved in identifying and degrading mRNAs with incorrectly formed 3'-ends within the nucleus. References: PMID:18644474 Sources: GOC:dgf, GOC:krc